{
  "term_id": "GO:0050808",
  "gene_symbol": "CNTN2",
  "gene_name": "Contactin-2",
  "gene": "UniProtKB:Q02246",
  "term_label": "synapse organization"
}